nuclear capsid assembly [GO:0039708] (biological process) Sources: VZ:1516 Relationships: is_a viral capsid assembly [GO:0019069]; occurs in host cell nucleus [GO:0042025] Definition: The assembly of a virus capsid that occurs in the nucleus. The assembly of large icosahedral shells for herpesviridae and adenoviridae requires structural proteins that act as chaperones for assembly.